{
  "gene_symbol": "TMEM70",
  "term_label": "Unknown molecular function",
  "gene_name": "Transmembrane protein 70, mitochondrial",
  "gene": "UniProtKB:Q9BUB7",
  "term_id": "UNKNOWN:0001"
}